brush border [GO:0005903] (cellular component) Definition: The dense covering of microvilli on the apical surface of an epithelial cell in tissues such as the intestine, kidney, and choroid plexus; the microvilli aid absorption by increasing the surface area of the cell. Relationships: is a type of GO:0098862; BFO_0000050 GO:0045177; has part microvillus [GO:0005902] Sources: GOC:sl, ISBN:0815316194